{
  "term_id": "GO:0005507",
  "term_label": "copper ion binding",
  "gene_symbol": "PRNP",
  "gene": "UniProtKB:P04156",
  "gene_name": "Major prion protein"
}